{
  "term_label": "Unknown molecular function",
  "gene_name": "Tax1-binding protein 1",
  "gene_symbol": "TAX1BP1",
  "gene": "UniProtKB:Q86VP1",
  "term_id": "UNKNOWN:0001"
}